{
  "term_label": "sensory perception of sound",
  "term_id": "GO:0007605",
  "gene": "UniProtKB:Q70EK8",
  "gene_name": "Inactive ubiquitin carboxyl-terminal hydrolase 53",
  "gene_symbol": "USP53"
}